{
  "gene": "UniProtKB:Q9Y3P9",
  "term_id": "UNKNOWN:0003",
  "gene_symbol": "RABGAP1",
  "term_label": "Unknown cellular component",
  "gene_name": "Rab GTPase-activating protein 1"
}